{
  "gene_symbol": "IFT27",
  "gene": "UniProtKB:Q9BW83",
  "gene_name": "Intraflagellar transport protein 27 homolog",
  "term_label": "GTPase activity",
  "term_id": "GO:0003924"
}